{
  "term_label": "cytoplasm",
  "gene": "UniProtKB:P11021",
  "gene_symbol": "HSPA5",
  "term_id": "GO:0005737",
  "gene_name": "Endoplasmic reticulum chaperone BiP"
}